{
  "term_label": "cation channel complex",
  "gene_name": "Short transient receptor potential channel 4",
  "gene": "UniProtKB:Q9UBN4",
  "gene_symbol": "TRPC4",
  "term_id": "GO:0034703"
}